{
  "gene_name": "Polyunsaturated fatty acid 5-lipoxygenase",
  "gene_symbol": "ALOX5",
  "term_label": "arachidonate metabolic process",
  "gene": "UniProtKB:P09917",
  "term_id": "GO:0019369"
}